olfactory bulb tufted cell development [GO:0061449] (biological process) Relationships: is a type of GO:0021884; is part of GO:0021772 Definition: The process whose specific outcome is the progression of an olfactory bulb tufted cell over time, from initial commitment of the cell to a specific fate, to the fully functional differentiated cell. Sources: GOC:dph